{
  "term_id": "UNKNOWN:0003",
  "term_label": "Unknown cellular component",
  "gene_name": "T cell receptor gamma variable 3",
  "gene": "UniProtKB:P03979",
  "gene_symbol": "TRGV3"
}